{
  "gene_name": "Potassium channel subfamily K member 15",
  "gene_symbol": "KCNK15",
  "gene": "UniProtKB:Q9H427",
  "term_id": "GO:0071805",
  "term_label": "potassium ion transmembrane transport"
}